VCB complex [GO:0030891] (cellular component) References: PMID:11865071 Sources: GOC:mah Relationships: is a type of GO:0000153 Definition: A protein complex that possesses ubiquitin ligase activity; the complex is usually pentameric; for example, in mammals the subunits are pVHL, elongin B, elongin C, cullin-2 (Cul2), and Rbx1. Also known as: VHL complex, pVHL-elongin C-elongin B complex, von Hippel-Lindau tumor suppressor complex